{
  "gene_name": "Zinc finger and BTB domain-containing protein 8B",
  "gene": "UniProtKB:Q8NAP8",
  "term_id": "GO:0006357",
  "term_label": "regulation of transcription by RNA polymerase II",
  "gene_symbol": "ZBTB8B"
}